{
  "gene": "UniProtKB:Q9NZA1",
  "term_label": "Unknown cellular component",
  "gene_symbol": "CLIC5",
  "term_id": "UNKNOWN:0003",
  "gene_name": "Chloride intracellular channel protein 5"
}